{
  "term_label": "DNA-binding transcription factor activity, RNA polymerase II-specific",
  "gene_name": "Transcription factor JunB",
  "gene_symbol": "JUNB",
  "gene": "UniProtKB:P17275",
  "term_id": "GO:0000981"
}